{
  "gene_symbol": "BCAN",
  "gene": "UniProtKB:Q96GW7",
  "term_label": "extracellular space",
  "term_id": "GO:0005615",
  "gene_name": "Brevican core protein"
}